{
  "gene_symbol": "SLC6A6",
  "gene_name": "Sodium- and chloride-dependent taurine transporter",
  "term_id": "GO:0042995",
  "gene": "UniProtKB:P31641",
  "term_label": "cell projection"
}